plastid-encoded plastid RNA polymerase complex [GO:0000427] (CC) Definition: An RNA polymerase complex containing polypeptides encoded by the plastid genome. Plastid-encoded DNA-directed RNA polymerases resemble eubacterial multisubunit RNA polymerases, with a core composed of alpha, beta, and beta-prime subunits. Some forms contain multiple additional subunits. An additional sigma factor subunit is required for promoter recognition. Sources: GOC:krc, GOC:mah, GOC:pj Relationships: is a type of DNA-directed RNA polymerase complex [GO:0000428]; is part of plastid [GO:0009536] Subtypes: plastid-encoded plastid RNA polymerase complex A [GO:0000343], plastid-encoded plastid RNA polymerase complex B [GO:0000344]